{
  "gene_symbol": "RAI2",
  "gene_name": "Retinoic acid-induced protein 2",
  "term_id": "GO:0005634",
  "gene": "UniProtKB:Q9Y5P3",
  "term_label": "nucleus"
}